{
  "gene_symbol": "TRGV1",
  "gene_name": "Probable non-functional T cell receptor gamma variable",
  "gene": "UniProtKB:A0A0A0MS02",
  "term_label": "Unknown molecular function",
  "term_id": "UNKNOWN:0001"
}